positive regulation of lateral motor column neuron migration [GO:1902078] (biological process) References: PMID:20711475 Sources: GOC:TermGenie, GOC:yaf Also known as: up regulation of lateral motor column neuron migration, up-regulation of lateral motor column neuron migration, upregulation of lateral motor column neuron migration, activation of lateral motor column neuron migration Relationships: is a type of regulation of lateral motor column neuron migration [GO:1902076]; is a type of positive regulation of motor neuron migration [GO:1905485]; positively regulates lateral motor column neuron migration [GO:0097477] Definition: Any process that activates or increases the frequency, rate or extent of lateral motor column neuron migration.